positive regulation of inositol biosynthetic process [GO:1900090] (biological process) Definition: Any process that activates or increases the frequency, rate or extent of inositol biosynthetic process. References: PMID:22307851 Sources: GOC:TermGenie Also known as: activation of inositol anabolism, activation of inositol biosynthesis, activation of inositol formation, activation of inositol synthesis, activation of vitamin Bh biosynthesis, activation of vitamin Bh biosynthetic process, positive regulation of inositol anabolism, positive regulation of inositol biosynthesis, positive regulation of inositol formation, positive regulation of inositol synthesis, positive regulation of vitamin Bh biosynthesis, positive regulation of vitamin Bh biosynthetic process, up regulation of inositol anabolism, up regulation of inositol biosynthesis, up regulation of inositol biosynthetic process, up regulation of inositol formation, up regulation of inositol synthesis, up regulation of vitamin Bh biosynthesis, up regulation of vitamin Bh biosynthetic process, up-regulation of inositol anabolism, up-regulation of inositol biosynthesis, up-regulation of inositol biosynthetic process, up-regulation of inositol formation, up-regulation of inositol synthesis, up-regulation of vitamin Bh biosynthesis, up-regulation of vitamin Bh biosynthetic process, upregulation of inositol anabolism, upregulation of inositol biosynthesis, upregulation of inositol biosynthetic process, upregulation of inositol formation, upregulation of inositol synthesis, upregulation of vitamin Bh biosynthesis, upregulation of vitamin Bh biosynthetic process, activation of inositol biosynthetic process, activation of myo-inositol biosynthesis, activation of myo-inositol biosynthetic process, positive regulation of myo-inositol biosynthesis, positive regulation of myo-inositol biosynthetic process, up regulation of myo-inositol biosynthesis, up regulation of myo-inositol biosynthetic process, up-regulation of myo-inositol biosynthesis, up-regulation of myo-inositol biosynthetic process, upregulation of myo-inositol biosynthesis, upregulation of myo-inositol biosynthetic process Relationships: is a type of regulation of inositol biosynthetic process [GO:1900088]; is a type of positive regulation of alcohol biosynthetic process [GO:1902932]; positively regulates inositol biosynthetic process [GO:0006021]